{
  "term_id": "GO:0034497",
  "gene_name": "WD repeat domain phosphoinositide-interacting protein 4",
  "term_label": "protein localization to phagophore assembly site",
  "gene_symbol": "WDR45",
  "gene": "UniProtKB:Q9Y484"
}